ribulose-bisphosphate carboxylase activity [GO:0016984] (molecular function) Definition: Catalysis of the reaction: 2 (2R)-3-phosphoglycerate + 2 H+ = CO2 + D-ribulose 1,5-bisphosphate + H2O. Also known as: D-ribulose 1,5-diphosphate carboxylase activity, D-ribulose-1,5-bisphosphate carboxylase activity, RuBP carboxylase activity, RuBisCO activity, diphosphoribulose carboxylase activity, ribulose 1,5-bisphosphate carboxylase activity, ribulose 1,5-bisphosphate carboxylase/oxygenase activity, ribulose 1,5-diphosphate carboxylase activity, ribulose 1,5-diphosphate carboxylase/oxygenase activity, ribulose bisphosphate carboxylase/oxygenase activity, ribulose diphosphate carboxylase activity, ribulose diphosphate carboxylase/oxygenase activity, carboxydismutase activity Sources: RHEA:23124 Regulation: positively regulated by GO:0046863 Relationships: is a type of carboxy-lyase activity [GO:0016831]